{
  "term_label": "Unknown molecular function",
  "gene_name": "Putative zinc finger protein 833",
  "gene_symbol": "ZNF833P",
  "term_id": "UNKNOWN:0001",
  "gene": "UniProtKB:Q6ZTB9"
}